R2/R5 cell differentiation [GO:0048054] (biological process) Definition: The process in which relatively unspecialized cells acquire the specialized features of R2 and R5 photoreceptors. An example of this process is found in Drosophila melanogaster. Relationships: is a type of compound eye photoreceptor cell differentiation [GO:0001751] Sources: GOC:jid